{
  "term_label": "plasma membrane",
  "term_id": "GO:0005886",
  "gene_name": "Olfactory receptor 7G3",
  "gene_symbol": "OR7G3",
  "gene": "UniProtKB:Q8NG95"
}